{
  "gene": "UniProtKB:Q9P2E9",
  "gene_symbol": "RRBP1",
  "gene_name": "Ribosome-binding protein 1",
  "term_label": "Unknown molecular function",
  "term_id": "UNKNOWN:0001"
}